peptidase activator activity involved in apoptotic process [GO:0016505] (molecular function) Definition: Binds to and increases the activity of a peptidase that is involved in the apoptotic process. Sources: GOC:BHF, GOC:mah, GOC:mtg_apoptosis, GOC:rl Also known as: apoptotic protease activator activity Relationships: is a type of peptidase activator activity [GO:0016504]; is part of apoptotic process [GO:0006915] Subtypes: cysteine-type endopeptidase activator activity involved in apoptotic process [GO:0008656]